fin development [GO:0033333] (biological process) Sources: GOC:dgh Relationships: is a type of GO:0048736 Definition: The process whose specific outcome is the progression of a fin over time, from its formation to the mature structure. Subtypes: medial fin development [GO:0033338], pectoral fin development [GO:0033339], pelvic fin development [GO:0033340]